{
  "gene_name": "G-protein coupled receptor 15",
  "term_id": "GO:0005886",
  "gene_symbol": "GPR15",
  "term_label": "plasma membrane",
  "gene": "UniProtKB:P49685"
}